{
  "gene_symbol": "NUDT3",
  "term_label": "bis(5'-adenosyl)-pentaphosphatase activity",
  "term_id": "GO:0034432",
  "gene_name": "Diphosphoinositol polyphosphate phosphohydrolase 1",
  "gene": "UniProtKB:O95989"
}